{
  "term_label": "neuronal cell body",
  "gene_name": "Double-stranded RNA-binding protein Staufen homolog 1",
  "gene_symbol": "STAU1",
  "gene": "UniProtKB:O95793",
  "term_id": "GO:0043025"
}